{
  "gene_symbol": "SPANXN5",
  "term_id": "UNKNOWN:0001",
  "term_label": "Unknown molecular function",
  "gene": "UniProtKB:Q5MJ07",
  "gene_name": "Sperm protein associated with the nucleus on the X chromosome N5"
}